{
  "term_id": "UNKNOWN:0002",
  "gene_symbol": "FAM90A13P",
  "gene": "UniProtKB:P0C7W8",
  "gene_name": "Putative protein FAM90A13P",
  "term_label": "Unknown biological process"
}